1,5-anhydro-D-fructose biosynthetic process [GO:1901803] (biological process) Definition: The chemical reactions and pathways resulting in the formation of 1,5-anhydro-D-fructose. Also known as: 1,5-anhydro-D-fructose anabolism, 1,5-anhydro-D-fructose biosynthesis, 1,5-anhydro-D-fructose formation, 1,5-anhydro-D-fructose synthesis Relationships: is_a ketone biosynthetic process [GO:0042181]; is a type of polyol biosynthetic process [GO:0046173]; is a type of monosaccharide biosynthetic process [GO:0046364]; is a type of epoxide metabolic process [GO:0097176]; is a type of ether biosynthetic process [GO:1901503] References: PMID:15716041 Sources: GOC:TermGenie, GOC:yaf, MetaCyc:PWY-6992, UniPathway:UPA00738